{
  "gene_name": "Annexin A10",
  "gene_symbol": "ANXA10",
  "gene": "UniProtKB:Q9UJ72",
  "term_id": "GO:0001786",
  "term_label": "phosphatidylserine binding"
}